acetylesterase activity [GO:0008126] (molecular function) Subtypes: sialate O-acetylesterase activity [GO:0001681], rhamnogalacturonan acetylesterase activity [GO:0046575] Relationships: is a type of short-chain carboxylesterase activity [GO:0034338] Sources: EC:3.1.1.6 Also known as: C-esterase (in animal tissues), chloroesterase, citrus acetylesterase, p-nitrophenyl acetate esterase, acetic ester hydrolase activity, acetic-ester acetylhydrolase activity Definition: Catalysis of the reaction: an acetic ester + H2O = an alcohol + acetate.